negative regulation of glomerulus development [GO:0090194] (biological process) Definition: Any process that decreases the rate, frequency or extent of glomerulus development, the progression of the glomerulus over time from its initial formation until its mature state. The glomerulus is a capillary tuft surrounded by Bowman's capsule in nephrons of the vertebrate kidney. Subtypes: negative regulation of metanephric glomerulus development [GO:0072299], GO:2000088 Relationships: is_a negative regulation of kidney development [GO:0090185]; is_a GO:0090192; negatively regulates glomerulus development [GO:0032835] Sources: GOC:dph, GOC:tb, GOC:yaf